{
  "gene_name": "Ubiquitin carboxyl-terminal hydrolase 17-like protein 12",
  "term_id": "GO:0005829",
  "gene": "UniProtKB:C9JPN9",
  "gene_symbol": "USP17L12",
  "term_label": "cytosol"
}